{
  "term_id": "UNKNOWN:0001",
  "gene_symbol": "WDR12",
  "gene": "UniProtKB:Q9GZL7",
  "gene_name": "Ribosome biogenesis protein WDR12",
  "term_label": "Unknown molecular function"
}